{
  "term_label": "regulation of actin filament polymerization",
  "term_id": "GO:0030833",
  "gene": "UniProtKB:Q9P2N2",
  "gene_symbol": "ARHGAP28",
  "gene_name": "Rho GTPase-activating protein 28"
}